{
  "term_label": "regulation of presynaptic cytosolic calcium ion concentration",
  "gene_symbol": "KCNH1",
  "term_id": "GO:0099509",
  "gene_name": "Potassium voltage-gated channel subfamily H member 1",
  "gene": "UniProtKB:O95259"
}